{
  "term_label": "membrane",
  "gene_symbol": "OR10J3",
  "term_id": "GO:0016020",
  "gene": "UniProtKB:Q5JRS4",
  "gene_name": "Olfactory receptor 10J3"
}